{
  "gene_symbol": "DEFB130A",
  "term_label": "extracellular space",
  "gene": "UniProtKB:P0DP74",
  "term_id": "GO:0005615",
  "gene_name": "Beta-defensin 130A"
}